regulation of starch biosynthetic process [GO:0010581] (biological process) Relationships: is_a regulation of glucan biosynthetic process [GO:0010962]; is a type of regulation of starch metabolic process [GO:2000904]; regulates starch biosynthetic process [GO:0019252] Subtypes: negative regulation of starch biosynthetic process [GO:7770012] Definition: An process which modulate the frequency, rate or extent of starch biosynthesis, the chemical reactions and pathways resulting in the formation of starch. Sources: GOC:tb